myosin XV complex [GO:0031485] (cellular component) Definition: A myosin complex containing a class XV myosin heavy chain and associated light chains. Myosin XV is single headed, and has a large extension (1200aa) at the N-terminus of the motor domain, two IQ motifs and a tail with a similar domain structure to that of the tail of myosin VII. References: PMID:10722873 Relationships: is a type of unconventional myosin complex [GO:0016461]